{
  "gene": "UniProtKB:Q8NGY3",
  "term_id": "GO:0016020",
  "gene_name": "Olfactory receptor 6K3",
  "term_label": "membrane",
  "gene_symbol": "OR6K3"
}